{
  "gene": "UniProtKB:Q8WWZ1",
  "term_id": "GO:0005125",
  "term_label": "cytokine activity",
  "gene_name": "Interleukin-1 family member 10",
  "gene_symbol": "IL1F10"
}